{
  "gene_name": "Dual specificity protein phosphatase CDC14A",
  "gene": "UniProtKB:Q9UNH5",
  "term_label": "microtubule cytoskeleton organization",
  "term_id": "GO:0000226",
  "gene_symbol": "CDC14A"
}